positive regulation of brown fat cell proliferation [GO:0070349] (biological process) Definition: Any process that activates or increases the rate or extent of brown fat cell proliferation. Relationships: is_a positive regulation of fat cell proliferation [GO:0070346]; is a type of regulation of brown fat cell proliferation [GO:0070347]; positively regulates brown fat cell proliferation [GO:0070342] Sources: GOC:mah, GOC:sl Also known as: positive regulation of brown adipocyte proliferation, positive regulation of brown adipose cell proliferation, up regulation of brown fat cell proliferation, up-regulation of brown fat cell proliferation, upregulation of brown fat cell proliferation, activation of brown fat cell proliferation, stimulation of brown fat cell proliferation